deoxyinosine metabolic process [GO:0046094] (biological process) Subtypes: deoxyinosine catabolic process [GO:0006149], GO:0046095 Relationships: is a type of GO:0046122 Sources: GOC:go_curators Also known as: deoxyinosine metabolism Definition: The chemical reactions and pathways involving deoxyinosine, hypoxanthine deoxyriboside.